{
  "gene_symbol": "GRIK2",
  "gene_name": "Glutamate receptor ionotropic, kainate 2",
  "term_id": "GO:0035249",
  "gene": "UniProtKB:Q13002",
  "term_label": "synaptic transmission, glutamatergic"
}